L-arabinitol 2-dehydrogenase activity [GO:0047002] (molecular function) Relationships: is a type of oxidoreductase activity, acting on the CH-OH group of donors, NAD or NADP as acceptor [GO:0016616] Sources: EC:1.1.1.13, RHEA:21356 Also known as: L-arabinitol 2-dehydrogenase (ribulose forming) activity Definition: Catalysis of the reaction: L-arabinitol + NAD+ = L-ribulose + H+ + NADH.